{
  "gene": "UniProtKB:P09493",
  "gene_name": "Tropomyosin alpha-1 chain",
  "gene_symbol": "TPM1",
  "term_id": "GO:0051015",
  "term_label": "actin filament binding"
}